negative regulation of cAMP/PKA signal transduction [GO:0141162] (biological process) Definition: Any process that stops, prevents or reduces the frequency, rate or extent of cAMP/PKA signal transduction. Relationships: is a type of GO:0141161; is a type of negative regulation of intracellular signal transduction [GO:1902532]; negatively regulates cAMP/PKA signal transduction [GO:0141156] Also known as: negative regulation of cAMP/PKA signaling References: PMID:17376027